{
  "term_id": "GO:0045165",
  "gene": "UniProtKB:P56704",
  "gene_symbol": "WNT3A",
  "term_label": "cell fate commitment",
  "gene_name": "Protein Wnt-3a"
}